{
  "gene_name": "Zinc finger protein 76",
  "gene": "UniProtKB:P36508",
  "term_label": "regulation of transcription by RNA polymerase II",
  "gene_symbol": "ZNF76",
  "term_id": "GO:0006357"
}